negative regulation of ripoptosome assembly involved in necroptotic process [GO:1902443] (biological process) References: PMID:21052097 Sources: GOC:TermGenie, GOC:dph, GOC:mtg_apoptosis Relationships: is a type of negative regulation of protein-containing complex assembly [GO:0031333]; is a type of regulation of ripoptosome assembly involved in necroptotic process [GO:1902442]; negatively regulates GO:1901026 Definition: Any process that stops, prevents or reduces the frequency, rate or extent of ripoptosome assembly involved in a necroptotic process. Also known as: down regulation of ripoptosome assembly involved in necroptosis, down-regulation of ripoptosome assembly involved in necroptosis, downregulation of ripoptosome assembly involved in necroptosis, inhibition of ripoptosome assembly involved in necroptosis, negative regulation of ripoptosome assembly involved in necroptosis